{
  "gene": "UniProtKB:O95343",
  "gene_name": "Homeobox protein SIX3",
  "term_label": "RNA polymerase II cis-regulatory region sequence-specific DNA binding",
  "gene_symbol": "SIX3",
  "term_id": "GO:0000978"
}